{
  "term_id": "GO:0042626",
  "term_label": "ATPase-coupled transmembrane transporter activity",
  "gene_name": "ATP-binding cassette sub-family D member 1",
  "gene_symbol": "ABCD1",
  "gene": "UniProtKB:P33897"
}